positive regulation of F-9775A biosynthetic process [GO:1900672] (biological process) Definition: Any process that activates or increases the frequency, rate or extent of F-9775A biosynthetic process. Sources: GOC:TermGenie, GOC:di Relationships: is a type of GO:1900670; is a type of positive regulation of polyketide biosynthetic process [GO:1900734]; RO_0002213 F-9775A biosynthetic process [GO:1900611] Also known as: activation of F-9775A anabolism, activation of F-9775A biosynthesis, activation of F-9775A formation, activation of F-9775A synthesis, positive regulation of F-9775A anabolism, positive regulation of F-9775A biosynthesis, positive regulation of F-9775A formation, positive regulation of F-9775A synthesis, up regulation of F-9775A anabolism, up regulation of F-9775A biosynthesis, up regulation of F-9775A biosynthetic process, up regulation of F-9775A formation, up regulation of F-9775A synthesis, up-regulation of F-9775A anabolism, up-regulation of F-9775A biosynthesis, up-regulation of F-9775A biosynthetic process, up-regulation of F-9775A formation, up-regulation of F-9775A synthesis, upregulation of F-9775A anabolism, upregulation of F-9775A biosynthesis, upregulation of F-9775A biosynthetic process, upregulation of F-9775A formation, upregulation of F-9775A synthesis, activation of F-9775A biosynthetic process